{
  "gene_name": "Leucine-rich repeat-containing protein 37B",
  "gene": "UniProtKB:Q96QE4",
  "term_label": "Unknown cellular component",
  "gene_symbol": "LRRC37B",
  "term_id": "UNKNOWN:0003"
}